{
  "term_id": "GO:0047498",
  "gene_symbol": "PLA2G2D",
  "gene_name": "Group IID secretory phospholipase A2",
  "term_label": "calcium-dependent phospholipase A2 activity",
  "gene": "UniProtKB:Q9UNK4"
}